{
  "gene_symbol": "TEX55",
  "gene_name": "Testis-specific expressed protein 55",
  "term_id": "GO:0005634",
  "term_label": "nucleus",
  "gene": "UniProtKB:Q96M34"
}